{
  "gene_symbol": "TKTL2",
  "gene_name": "Transketolase-like protein 2",
  "gene": "UniProtKB:Q9H0I9",
  "term_label": "cytosol",
  "term_id": "GO:0005829"
}